{
  "term_label": "Unknown cellular component",
  "term_id": "UNKNOWN:0003",
  "gene_name": "Transmembrane protein 205",
  "gene": "UniProtKB:Q6UW68",
  "gene_symbol": "TMEM205"
}